detection of tumor cell [GO:0002355] (biological process) Definition: The series of events in which a stimulus from a tumor cell is received and converted into a molecular signal. Relationships: is a type of response to tumor cell [GO:0002347]; is a type of GO:0009595 References: PMID:16730260 Sources: GOC:add, ISBN:0781735149